{
  "term_id": "GO:0034364",
  "term_label": "high-density lipoprotein particle",
  "gene_name": "Apolipoprotein C-IV",
  "gene_symbol": "APOC4",
  "gene": "UniProtKB:P55056"
}